hydrogen sulfide metabolic process [GO:0070813] (biological process) Relationships: is a type of GO:0006790 Sources: GOC:mah Also known as: hydrogen sulfide metabolism, hydrogen sulphide metabolic process, hydrogen sulphide metabolism Definition: The chemical reactions and pathways involving hydrogen sulfide, H2S. Subtypes: hydrogen sulfide biosynthetic process [GO:0070814]